interstrand cross-link repair [GO:0036297] (biological process) Definition: Removal of a DNA interstrand crosslink (a covalent attachment of DNA bases on opposite strands of the DNA) and restoration of the DNA. DNA interstrand crosslinks occur when both strands of duplex DNA are covalently tethered together (e.g. by an exogenous or endogenous agent), thus preventing the strand unwinding necessary for essential DNA functions such as transcription and replication. Relationships: is a type of GO:0006281 Subtypes: recombinational interstrand cross-link repair [GO:0036298], non-recombinational interstrand cross-link repair [GO:0036299] References: PMID:16464006, PMID:22064477 Sources: GOC:vw Also known as: ICL repair